{
  "gene_symbol": "HOXC5",
  "term_id": "GO:0006357",
  "gene": "UniProtKB:Q00444",
  "gene_name": "Homeobox protein Hox-C5",
  "term_label": "regulation of transcription by RNA polymerase II"
}